alpha9-beta1 integrin-ADAM3 complex [GO:0071054] (CC) References: PMID:11882657 Also known as: ITGA9-ITGB1-ADAM3 complex Definition: A protein complex that consists of an alpha9-beta1 integrin complex bound to the transmembrane metallopeptidase ADAM3. Relationships: is a type of plasma membrane protein complex [GO:0098797]